far-red light signaling pathway [GO:0010018] (biological process) Relationships: is a type of red or far-red light signaling pathway [GO:0010017]; is a type of cellular response to far red light [GO:0071490] Sources: GOC:lr, GOC:mtg_far_red, GOC:sm Definition: The series of molecular signals initiated upon sensing of far red light by a photoreceptor molecule. Far red light is electromagnetic radiation of wavelength 700-800nm. An example of this response is seen at the beginning of many plant species developmental stages. These include germination, and the point when cotyledon expansion is triggered. In certain species these processes take place in response to absorption of red light by the pigment molecule phytochrome, but the signal can be reversed by exposure to far red light. During the initial phase the phytochrome molecule is only present in the red light absorbing form, but on absorption of red light it changes to a far red light absorbing form, triggering progress through development. An immediate short period of exposure to far red light entirely returns the pigment to its initial state and prevents triggering of the developmental process. A thirty minute break between red and subsequent far red light exposure renders the red light effect irreversible, and development then occurs regardless of whether far red light exposure subsequently occurs. Also known as: far red light signalling pathway, far red signaling pathway, far-red light signal transduction